response to gibberellin [GO:0009739] (biological process) Definition: Any process that results in a change in state or activity of a cell or an organism (in terms of movement, secretion, enzyme production, gene expression, etc.) as a result of a gibberellin stimulus. Sources: GOC:jl Also known as: response to gibberellin stimulus, response to gibberellic acid stimulus Relationships: is a type of GO:0009725; is a type of response to lipid [GO:0033993]; is a type of response to oxygen-containing compound [GO:1901700] Subtypes: detection of gibberellic acid stimulus [GO:0009728], cellular response to gibberellin stimulus [GO:0071370]